{
  "gene_name": "Carboxy-terminal domain RNA polymerase II polypeptide A small phosphatase 2",
  "gene": "UniProtKB:O14595",
  "term_id": "GO:0008420",
  "term_label": "RNA polymerase II CTD heptapeptide repeat phosphatase activity",
  "gene_symbol": "CTDSP2"
}